response to cytokinin [GO:0009735] (biological process) Also known as: response to cytokinin stimulus Relationships: is a type of response to hormone [GO:0009725] Subtypes: detection of cytokinin stimulus [GO:0009722], GO:0071368 Sources: GOC:jl Definition: Any process that results in a change in state or activity of a cell or an organism (in terms of movement, secretion, enzyme production, gene expression, etc.) as a result of a cytokinin stimulus.